{
  "term_label": "complement receptor activity",
  "gene_symbol": "FPR3",
  "gene_name": "N-formyl peptide receptor 3",
  "gene": "UniProtKB:P25089",
  "term_id": "GO:0004875"
}